{
  "term_label": "muscle contraction",
  "gene_symbol": "MYH3",
  "gene": "UniProtKB:P11055",
  "term_id": "GO:0006936",
  "gene_name": "Myosin-3"
}